positive regulation of galactoglucomannan catabolic process [GO:2000914] (biological process) Sources: GOC:mengo_curators Also known as: positive regulation of galactoglucomannan catabolism Definition: Any process that activates or increases the frequency, rate or extent of galactoglucomannan catabolic process. Relationships: is a type of GO:0009896; is a type of positive regulation of macromolecule metabolic process [GO:0010604]; is a type of positive regulation of carbohydrate metabolic process [GO:0045913]; is a type of regulation of galactoglucomannan catabolic process [GO:2000912]; positively regulates galactoglucomannan catabolic process [GO:2000885]